{
  "gene_symbol": "USP17L30",
  "term_label": "nucleus",
  "gene": "UniProtKB:Q0WX57",
  "term_id": "GO:0005634",
  "gene_name": "Ubiquitin carboxyl-terminal hydrolase 17-like protein 24"
}